{
  "gene_name": "Muscle, skeletal receptor tyrosine-protein kinase",
  "gene": "UniProtKB:O15146",
  "gene_symbol": "MUSK",
  "term_label": "Wnt-protein binding",
  "term_id": "GO:0017147"
}